{
  "gene_name": "Protein-tyrosine kinase 6",
  "gene": "UniProtKB:Q13882",
  "gene_symbol": "PTK6",
  "term_id": "GO:0004715",
  "term_label": "non-membrane spanning protein tyrosine kinase activity"
}